{
  "gene_name": "Carboxypeptidase B2",
  "term_label": "proteolysis",
  "gene_symbol": "CPB2",
  "term_id": "GO:0006508",
  "gene": "UniProtKB:Q96IY4"
}